{
  "gene": "UniProtKB:Q8TBZ5",
  "gene_symbol": "ZNF502",
  "term_label": "RNA polymerase II cis-regulatory region sequence-specific DNA binding",
  "term_id": "GO:0000978",
  "gene_name": "Zinc finger protein 502"
}